columella [GO:0043674] (cellular component) Relationships: is_a cellular anatomical structure [GO:0110165]; is part of sexine [GO:0043673] Definition: A rod-like element of the sexine and ectexine, supporting either the tectum (the layer of sexine which forms a roof over the columella), or supporting a caput (an architectural element on top of a columella). Also known as: sexine 1 Sources: https://en.wikipedia.org/wiki/Columella_(botany)